fat cell proliferation [GO:0070341] (biological process) Regulation: regulated by regulation of fat cell proliferation [GO:0070344]; RO_0002212 by negative regulation of fat cell proliferation [GO:0070345]; positively regulated by positive regulation of fat cell proliferation [GO:0070346] Also known as: adipocyte proliferation, adipose cell proliferation Sources: GOC:mah, GOC:sl Relationships: is a type of GO:0008283 Subtypes: brown fat cell proliferation [GO:0070342], white fat cell proliferation [GO:0070343] Definition: The multiplication or reproduction of fat cells by cell division, resulting in the expansion of their population. A fat cell is an animal connective tissue cell specialized for the synthesis and storage of fat.